{
  "term_id": "GO:0035666",
  "term_label": "TRIF-dependent toll-like receptor signaling pathway",
  "gene": "UniProtKB:Q8IUC6",
  "gene_name": "TIR domain-containing adapter molecule 1",
  "gene_symbol": "TICAM1"
}